protein-N(PI)-phosphohistidine-maltose phosphotransferase system transporter activity [GO:0022873] (molecular function) Relationships: is a type of maltose transmembrane transporter activity [GO:0005363]; is a type of GO:0008982 Sources: GOC:mtg_transport, ISBN:0815340729 Definition: Catalysis of the PEP-dependent, phosphoryl transfer-driven transport of substances across a membrane. The transport happens by catalysis of the reaction: protein N-phosphohistidine + maltose(out) = protein histidine + maltose phosphate(in). This differs from primary and secondary active transport in that the solute is modified during transport. Also known as: maltose PTS transporter activity